{
  "gene_name": "Protein FAM25G",
  "gene_symbol": "FAM25G",
  "term_label": "Unknown biological process",
  "gene": "UniProtKB:B3EWG6",
  "term_id": "UNKNOWN:0002"
}